{
  "gene": "UniProtKB:Q6Q795",
  "term_id": "UNKNOWN:0003",
  "term_label": "Unknown cellular component",
  "gene_symbol": "Q6Q795",
  "gene_name": "Putative viral protein-binding protein C1"
}